{
  "gene_symbol": "CEBPZOS",
  "gene_name": "Protein CEBPZOS",
  "gene": "UniProtKB:A8MTT3",
  "term_id": "UNKNOWN:0002",
  "term_label": "Unknown biological process"
}